negative regulation of progesterone biosynthesis involved in luteolysis [GO:0061363] (biological process) Relationships: is a type of negative regulation of progesterone biosynthetic process [GO:2000183]; is part of luteolysis [GO:0001554] Sources: GOC:dph Also known as: functional luteolysis Definition: Any process that decreases the rate, frequency or extent of the biosynthesis of progesterone biosynthesis that contributes to luteolysis.